{
  "gene": "UniProtKB:P51160",
  "gene_symbol": "PDE6C",
  "gene_name": "Cone cGMP-specific 3',5'-cyclic phosphodiesterase subunit alpha'",
  "term_label": "3',5'-cyclic-AMP phosphodiesterase activity",
  "term_id": "GO:0004115"
}